{
  "term_id": "GO:0004198",
  "gene": "UniProtKB:A8MX76",
  "gene_symbol": "CAPN14",
  "gene_name": "Calpain-14",
  "term_label": "calcium-dependent cysteine-type endopeptidase activity"
}